{
  "gene_name": "Tumor necrosis factor ligand superfamily member 4",
  "term_label": "inflammatory response",
  "gene_symbol": "TNFSF4",
  "term_id": "GO:0006954",
  "gene": "UniProtKB:P23510"
}